{
  "gene_name": "High affinity cationic amino acid transporter 1",
  "gene": "UniProtKB:P30825",
  "term_id": "GO:0005886",
  "term_label": "plasma membrane",
  "gene_symbol": "SLC7A1"
}